{
  "gene_symbol": "DAXX",
  "gene_name": "Death domain-associated protein 6",
  "gene": "UniProtKB:Q9UER7",
  "term_id": "GO:0016605",
  "term_label": "PML body"
}